{
  "gene_symbol": "IGKV1-37",
  "gene": "UniProtKB:A0A075B6S9",
  "term_id": "GO:0019814",
  "gene_name": "Probable non-functional immunoglobulinn kappa variable 1-37",
  "term_label": "immunoglobulin complex"
}